{
  "gene_symbol": "WWC2",
  "term_id": "GO:0005737",
  "gene_name": "Protein WWC2",
  "term_label": "cytoplasm",
  "gene": "UniProtKB:Q6AWC2"
}